{
  "gene_symbol": "CCDC140",
  "gene_name": "Coiled-coil domain-containing protein 140",
  "term_id": "UNKNOWN:0001",
  "term_label": "Unknown molecular function",
  "gene": "UniProtKB:Q96MF4"
}